{
  "term_label": "D1 dopamine receptor binding",
  "gene_name": "Beta-arrestin-2",
  "gene": "UniProtKB:P32121",
  "term_id": "GO:0031748",
  "gene_symbol": "ARRB2"
}